cell wall (1->3)-beta-D-glucan metabolic process [GO:0034407] (biological process) Relationships: is a type of GO:0006074; is a type of cell wall beta-glucan metabolic process [GO:0034406] Also known as: cell wall 1,3-beta-glucan metabolic process, cell wall 1,3-beta-D-glucan metabolic process, cell wall 1,3-beta-glucan metabolism, cell wall beta-1,3 glucan metabolic process, cell wall beta-1,3 glucan metabolism Definition: The chemical reactions and pathways involving (1->3)-beta-D-glucans, compounds composed of glucose residues linked by (1->3)-beta-D-glucosidic bonds, found in the walls of cells. Sources: GOC:mah Subtypes: GO:0034411, GO:0071969